negative regulation of natural killer cell chemotaxis [GO:2000502] (biological process) Sources: GOC:BHF Relationships: is a type of negative regulation of lymphocyte chemotaxis [GO:1901624]; is a type of GO:2000501; negatively regulates natural killer cell chemotaxis [GO:0035747] Definition: Any process that stops, prevents or reduces the frequency, rate or extent of natural killer cell chemotaxis.